ribonucleoside diphosphate catabolic process [GO:0009191] (biological process) Also known as: ribonucleoside diphosphate breakdown, ribonucleoside diphosphate catabolism, ribonucleoside diphosphate degradation Relationships: is a type of nucleoside diphosphate catabolic process [GO:0009134]; is a type of ribonucleoside diphosphate metabolic process [GO:0009185] Definition: The chemical reactions and pathways resulting in the breakdown of a ribonucleoside diphosphate, a compound consisting of a nucleobase linked to a ribose sugar esterified with diphosphate on the sugar. Subtypes: purine ribonucleoside diphosphate catabolic process [GO:0009181], pyrimidine ribonucleoside diphosphate catabolic process [GO:0009195] Sources: GOC:go_curators, ISBN:0198506732